{
  "gene_symbol": "A6NL46",
  "term_label": "Unknown cellular component",
  "term_id": "UNKNOWN:0003",
  "gene": "UniProtKB:A6NL46",
  "gene_name": "Putative UPF0607 protein ENSP00000332738"
}